{
  "term_label": "protein-folding chaperone binding",
  "gene": "UniProtKB:Q5SXM8",
  "gene_name": "DNL-type zinc finger protein",
  "term_id": "GO:0051087",
  "gene_symbol": "DNLZ"
}